{
  "gene": "UniProtKB:Q96CM3",
  "term_id": "GO:0000455",
  "gene_symbol": "RPUSD4",
  "term_label": "enzyme-directed rRNA pseudouridine synthesis",
  "gene_name": "Pseudouridylate synthase RPUSD4, mitochondrial"
}